{
  "term_label": "protein polyubiquitination",
  "gene_name": "Ubiquitin-conjugating enzyme E2 T",
  "term_id": "GO:0000209",
  "gene_symbol": "UBE2T",
  "gene": "UniProtKB:Q9NPD8"
}